{
  "gene": "UniProtKB:Q8TB96",
  "gene_name": "T-cell immunomodulatory protein",
  "term_label": "Unknown molecular function",
  "term_id": "UNKNOWN:0001",
  "gene_symbol": "ITFG1"
}